cerebral cortex GABAergic interneuron fate commitment [GO:0021893] (biological process) Definition: The process in which the developmental fate of a neuroblast becomes restricted such that it will develop into a GABAergic interneuron residing in the cerebral cortex. Relationships: is a type of GO:0048663; is part of cerebral cortex GABAergic interneuron differentiation [GO:0021892] References: PMID:12626695 Sources: GOC:cls, GOC:dgh, GOC:dph, GOC:jid, GO_REF:0000021